{
  "gene_name": "26S proteasome regulatory subunit 8",
  "gene": "UniProtKB:P62195",
  "term_id": "GO:0036402",
  "gene_symbol": "PSMC5",
  "term_label": "proteasome-activating activity"
}